{
  "gene_symbol": "CCN3",
  "gene": "UniProtKB:P48745",
  "gene_name": "CCN family member 3",
  "term_id": "GO:0007155",
  "term_label": "cell adhesion"
}